{
  "gene": "UniProtKB:Q9P253",
  "term_label": "lysosome organization",
  "gene_name": "Vacuolar protein sorting-associated protein 18 homolog",
  "term_id": "GO:0007040",
  "gene_symbol": "VPS18"
}